late endosome to Golgi transport [GO:0034499] (biological process) Sources: GOC:rb Also known as: PVE to Golgi transport, prevacuolar endosome to Golgi transport Definition: The directed movement of substances from late endosomes to the Golgi. Relationships: is a type of retrograde transport, endosome to Golgi [GO:0042147]; is a type of Golgi vesicle transport [GO:0048193]; occurs in cytoplasm [GO:0005737]